positive regulation of ion transmembrane transporter activity [GO:0032414] (BP) Definition: Any process that activates or increases the activity of an ion transporter. Sources: GOC:mah, GOC:tb Also known as: positive regulation of ion transporter activity, up regulation of ion transporter activity, up-regulation of ion transporter activity, upregulation of ion transporter activity, activation of ion transporter activity, stimulation of ion transporter activity Relationships: is a type of GO:0022898; is a type of positive regulation of transporter activity [GO:0032411]; is a type of positive regulation of monoatomic ion transmembrane transport [GO:0034767]; positively regulates monoatomic ion transmembrane transporter activity [GO:0015075] Subtypes: positive regulation of anion channel activity [GO:1901529], positive regulation of ATPase-coupled calcium transmembrane transporter activity [GO:1901896], GO:1904960, positive regulation of sodium ion transmembrane transporter activity [GO:2000651], positive regulation of AMPA receptor activity [GO:2000969], positive regulation of cation channel activity [GO:2001259]